{
  "gene_symbol": "PNLIPRP1",
  "gene_name": "Inactive pancreatic lipase-related protein 1",
  "term_label": "high-density lipoprotein particle remodeling",
  "gene": "UniProtKB:P54315",
  "term_id": "GO:0034375"
}